{
  "gene": "UniProtKB:Q9UIJ5",
  "gene_name": "Palmitoyltransferase ZDHHC2",
  "gene_symbol": "ZDHHC2",
  "term_id": "GO:0006612",
  "term_label": "protein targeting to membrane"
}